adenyl-nucleotide exchange factor activity [GO:0000774] (molecular function) Definition: Binds to and stimulates the hydrolysis and exchange of adenyl nucleotides by other proteins. Relationships: is a type of ATPase regulator activity [GO:0060590]; negatively regulates GO:0043531; positively regulates GO:0005524 Sources: GOC:kd